{
  "term_id": "UNKNOWN:0002",
  "gene_name": "F-box_WD repeat-containing protein 2",
  "term_label": "Unknown biological process",
  "gene_symbol": "FBXW2",
  "gene": "UniProtKB:Q9UKT8"
}